GTPase activating protein binding [GO:0032794] (molecular function) Definition: Binding to a GTPase activating protein. Sources: GOC:nln Also known as: GAP binding Relationships: is a type of protein binding [GO:0005515]